regulation of cytokinesis, actomyosin contractile ring assembly [GO:2000431] (biological process) Definition: Any process that modulates the frequency, rate or extent of cytokinesis, actomyosin contractile ring assembly. Sources: GOC:obol Also known as: regulation of contractile ring assembly Subtypes: regulation of mitotic actomyosin contractile ring assembly [GO:1903499], negative regulation of cytokinesis, actomyosin contractile ring assembly [GO:2000432], GO:2000433 Relationships: is a type of regulation of cytokinetic process [GO:0032954]; is a type of regulation of cellular component biogenesis [GO:0044087]; is a type of regulation of actomyosin structure organization [GO:0110020]; regulates GO:0000915